regulation of macrophage migration [GO:1905521] (biological process) Relationships: is a type of GO:0071675; regulates macrophage migration [GO:1905517] Subtypes: regulation of macrophage chemotaxis [GO:0010758], regulation of microglial cell migration [GO:1904139], negative regulation of macrophage migration [GO:1905522], GO:1905523 Definition: Any process that modulates the frequency, rate or extent of macrophage migration. References: PMID:25749876 Sources: GOC:TermGenie, GO_REF:0000058